FK506 binding [GO:0005528] (molecular function) Also known as: FK506-sensitive peptidyl-prolyl cis-trans isomerase Sources: GOC:jl Definition: Binding to a 23-membered macrolide lactone FK506. Relationships: is a type of macrolide binding [GO:0005527]; is a type of amide binding [GO:0033218]